germline ring canal [GO:0045172] (cellular component) References: PMID:9635420, PMID:9655801 Sources: GOC:mtg_sensu Relationships: is a type of intercellular bridge [GO:0045171] Subtypes: male germline ring canal [GO:0035323], female germline ring canal [GO:0035324] Definition: Germline specific intercellular bridge. During cyst formation in insects, ring canals interconnect the cells of the cyst, facilitating the passage of cytoplasmic components between cells.